{
  "gene_name": "Homeobox protein Hox-D3",
  "term_id": "GO:0009952",
  "gene_symbol": "HOXD3",
  "gene": "UniProtKB:P31249",
  "term_label": "anterior/posterior pattern specification"
}